rDNA heterochromatin formation [GO:0000183] (biological process) Regulation: regulated by regulation of rDNA heterochromatin formation [GO:0061187]; negatively regulated by negative regulation of rDNA heterochromatin formation [GO:0061188]; RO_0002213 by GO:2000749 Relationships: is a type of facultative heterochromatin formation [GO:0140718]; is part of nucleolar chromatin organization [GO:1990700] References: PMID:10219245 Also known as: chromatin silencing at ribosomal DNA, heterochromatic silencing at rDNA, rDNA chromatin silencing, rDNA heterochromatin assembly, chromatin silencing at rDNA Definition: The formation of heterochromatin at ribosomal DNA, characterized by the modified histone H3K9me3.